{
  "term_id": "GO:0055085",
  "term_label": "transmembrane transport",
  "gene": "UniProtKB:O15439",
  "gene_name": "ATP-binding cassette sub-family C member 4",
  "gene_symbol": "ABCC4"
}